cilium movement [GO:0003341] (biological process) Relationships: is a type of GO:0007018 Also known as: microtubule-based flagellum movement, flagellar movement, flagellum movement, ciliary motility, cilium beating, flagellar motility Sources: GOC:dph, GOC:jl Subtypes: epithelial cilium movement involved in extracellular fluid movement [GO:0003351], cilium movement involved in cell motility [GO:0060294] Note: Note that we deem cilium and microtubule-based flagellum to be equivalent. Regulation: RO_0002211 by regulation of cilium movement [GO:0003352]; positively regulated by GO:0003353; negatively regulated by negative regulation of cilium movement [GO:0003354] Definition: The directed, self-propelled movement of a cilium.